old cell pole [GO:1990901] (cellular component) References: PMID:10231492, PMID:8226658 Sources: GOC:jh2 Definition: The cell pole distal from the most recent cell division. Relationships: is a type of GO:0060187